{
  "term_label": "cytoplasm",
  "gene": "UniProtKB:Q9NNZ6",
  "gene_symbol": "PRM3",
  "gene_name": "Protamine-3",
  "term_id": "GO:0005737"
}